{
  "gene": "UniProtKB:P25092",
  "term_label": "guanylate cyclase activity",
  "gene_name": "Guanylyl cyclase C",
  "gene_symbol": "GUCY2C",
  "term_id": "GO:0004383"
}